{
  "term_id": "GO:0005886",
  "term_label": "plasma membrane",
  "gene": "UniProtKB:Q9P241",
  "gene_symbol": "ATP10D",
  "gene_name": "Phospholipid-transporting ATPase VD"
}